{
  "gene_name": "Dipeptidyl peptidase 2",
  "gene_symbol": "DPP7",
  "gene": "UniProtKB:Q9UHL4",
  "term_label": "Unknown biological process",
  "term_id": "UNKNOWN:0002"
}